{
  "term_id": "UNKNOWN:0001",
  "gene_name": "T cell receptor beta joining 1-6",
  "gene_symbol": "TRBJ1-6",
  "gene": "UniProtKB:A0A0J9YWX3",
  "term_label": "Unknown molecular function"
}